{
  "gene_symbol": "INPP5D",
  "gene": "UniProtKB:Q92835",
  "term_label": "Unknown molecular function",
  "gene_name": "Phosphatidylinositol 3,4,5-trisphosphate 5-phosphatase 1",
  "term_id": "UNKNOWN:0001"
}